{
  "gene_name": "C-type lectin domain family 7 member A",
  "term_label": "phagocytosis, recognition",
  "gene_symbol": "CLEC7A",
  "gene": "UniProtKB:Q9BXN2",
  "term_id": "GO:0006910"
}